{
  "gene_name": "Protein S100-A6",
  "term_label": "S100 protein binding",
  "gene_symbol": "S100A6",
  "term_id": "GO:0044548",
  "gene": "UniProtKB:P06703"
}